{
  "term_label": "Unknown molecular function",
  "term_id": "UNKNOWN:0001",
  "gene_symbol": "CNTRL",
  "gene": "UniProtKB:Q7Z7A1",
  "gene_name": "Centriolin"
}